{
  "term_label": "adenylate cyclase-inhibiting serotonin receptor signaling pathway",
  "gene_name": "5-hydroxytryptamine receptor 1A",
  "term_id": "GO:0007198",
  "gene_symbol": "HTR1A",
  "gene": "UniProtKB:P08908"
}